{
  "gene": "UniProtKB:Q9Y6K9",
  "term_id": "GO:0008385",
  "gene_symbol": "IKBKG",
  "term_label": "IkappaB kinase complex",
  "gene_name": "NF-kappa-B essential modulator"
}